{
  "term_label": "chordate embryonic development",
  "gene_symbol": "BRCA1",
  "term_id": "GO:0043009",
  "gene": "UniProtKB:P38398",
  "gene_name": "Breast cancer type 1 susceptibility protein"
}